phagolysosome assembly involved in apoptotic cell clearance [GO:0090387] (biological process) Definition: The process in which a phagosome, a vesicle formed by phagocytosis, fuses with a lysosome as a part of apoptotic cell clearance. Sources: GOC:kmv, GOC:tb Relationships: is a type of GO:0001845; is part of GO:0090386